{
  "gene_symbol": "SQLE",
  "gene_name": "Squalene monooxygenase",
  "term_id": "GO:0005783",
  "gene": "UniProtKB:Q14534",
  "term_label": "endoplasmic reticulum"
}